mannan polymerase complex [GO:0000136] (cellular component) Also known as: alpha-1,6-mannosyltransferase complex References: PMID:10037752, PMID:11095735, PMID:18083825 Sources: GOC:mcc Subtypes: mannan polymerase II complex [GO:0140497], mannan polymerase I complex [GO:0140498] Definition: A protein complex with alpha-(1->6)-mannosyltransferase activity, located in the cis Golgi membrane; adds mannan to N-linked glycans on proteins. Relationships: is_a mannosyltransferase complex [GO:0031501]; is a type of membrane protein complex [GO:0098796]; is part of Golgi cis cisterna [GO:0000137]; BFO_0000050 Golgi membrane [GO:0000139]